{
  "gene_symbol": "NEURL1",
  "term_label": "plasma membrane",
  "term_id": "GO:0005886",
  "gene_name": "E3 ubiquitin-protein ligase NEURL1",
  "gene": "UniProtKB:O76050"
}